hexuronate transmembrane transport [GO:0015736] (biological process) Subtypes: galacturonate transmembrane transport [GO:0015737], GO:0015738 Sources: GOC:ai, ISBN:0198506732 Also known as: hexuronate transport Definition: The process in which hexuronate is transported across a lipid bilayer, from one side of a membrane to the other. A hexuronate is any monocarboxylic acid derived from a hexose by oxidation of C-6. Relationships: is a type of uronic acid transmembrane transport [GO:0015735]